tRNA (N(6)-L-threonylcarbamoyladenosine(37)-C(2))-methylthiotransferase activity [GO:0035598] (molecular function) Definition: Catalysis of the reaction: N(6)-L-threonylcarbamoyladenosine(37) in tRNA + [sulfur carrier]-SH + AH2 + 2 S-adenosyl-L-methionine = 2-methylsulfanyl-N(6)-L-threonylcarbamoyladenosine(37) in tRNA + [sulfur carrier]-H + 5'-deoxyadenosine + L-methionine + A + S-adenosyl-L-homocysteine + 2 H+. Relationships: is a type of methylthiotransferase activity [GO:0035596]; is a type of catalytic activity, acting on a tRNA [GO:0140101]; is part of tRNA methylthiolation [GO:0035600] References: PMID:20472640, PMID:20584901 Sources: RHEA:37075 Also known as: N6-threonylcarbomyladenosine methylthiotransferase activity, t6A methylthiotransferase activity